{
  "gene_symbol": "WFDC3",
  "gene": "UniProtKB:Q8IUB2",
  "gene_name": "WAP four-disulfide core domain protein 3",
  "term_id": "GO:0019731",
  "term_label": "antibacterial humoral response"
}